regulation of filamentous growth of a population of unicellular organisms in response to neutral pH [GO:1900440] (biological process) Sources: GOC:TermGenie, GOC:di Subtypes: GO:1900441, positive regulation of filamentous growth of a population of unicellular organisms in response to neutral pH [GO:1900442] Relationships: is a type of GO:1900741; regulates GO:0036178 Definition: Any process that modulates the frequency, rate or extent of filamentous growth of a population of unicellular organisms in response to neutral pH.